{
  "gene": "UniProtKB:P53420",
  "gene_name": "Collagen alpha-4(IV) chain",
  "term_label": "glomerular basement membrane development",
  "term_id": "GO:0032836",
  "gene_symbol": "COL4A4"
}